{
  "gene_symbol": "EYA3",
  "gene_name": "Eyes absent homolog 3",
  "term_label": "nucleus",
  "term_id": "GO:0005634",
  "gene": "UniProtKB:Q99504"
}